laminin complex [GO:0043256] (cellular component) References: PMID:10842354 Sources: GOC:jl Relationships: is_a protein-containing complex [GO:0032991]; BFO_0000050 basement membrane [GO:0005604] Subtypes: GO:0005606, laminin-2 complex [GO:0005607], laminin-3 complex [GO:0005608], GO:0005609, GO:0005610, laminin-6 complex [GO:0005611], laminin-7 complex [GO:0005612], laminin-8 complex [GO:0043257], laminin-9 complex [GO:0043258], GO:0043259, laminin-11 complex [GO:0043260], laminin-12 complex [GO:0043261], GO:0061801, laminin-14 complex [GO:1990338], laminin-522 complex [GO:1990339], GO:1990340 Definition: A large, extracellular glycoprotein complex composed of three different polypeptide chains, alpha, beta and gamma. Provides an integral part of the structural scaffolding of basement membranes.